{
  "gene_symbol": "MT-ND4",
  "gene_name": "NADH-ubiquinone oxidoreductase chain 4",
  "term_label": "respiratory chain complex I",
  "gene": "UniProtKB:P03905",
  "term_id": "GO:0045271"
}